{
  "gene": "UniProtKB:Q96BY6",
  "term_id": "GO:0030334",
  "gene_name": "Dedicator of cytokinesis protein 10",
  "gene_symbol": "DOCK10",
  "term_label": "regulation of cell migration"
}